{
  "gene": "UniProtKB:Q1W4C9",
  "gene_name": "Serine protease inhibitor Kazal-type 13",
  "term_label": "Unknown molecular function",
  "term_id": "UNKNOWN:0001",
  "gene_symbol": "SPINK13"
}